{
  "term_id": "GO:0005737",
  "gene": "UniProtKB:Q99932",
  "gene_symbol": "SPAG8",
  "term_label": "cytoplasm",
  "gene_name": "Sperm-associated antigen 8"
}